follicular fluid formation in ovarian follicle antrum involved in distinct antral spaces stage [GO:0003004] (BP) Also known as: follicular fluid formation in ovarian follicle antrum during distinct antral spaces stage Sources: GOC:dph, GOC:isa_complete Definition: The menstrual cycle process in which one central cavity separating the oocyte/cumulus complex from mural granulosa and theca cells is formed as part of the antral spaces stage of oogenesis. Relationships: is a type of follicular fluid formation in ovarian follicle antrum [GO:0001548]; is part of distinct antral spaces stage [GO:0048164]